{
  "gene_name": "Serine hydrolase RBBP9",
  "term_label": "Unknown molecular function",
  "term_id": "UNKNOWN:0001",
  "gene_symbol": "RBBP9",
  "gene": "UniProtKB:O75884"
}